{
  "gene_symbol": "CMIP",
  "term_label": "Unknown biological process",
  "gene_name": "C-Maf-inducing protein",
  "term_id": "UNKNOWN:0002",
  "gene": "UniProtKB:Q8IY22"
}